{
  "term_id": "GO:0005737",
  "gene_symbol": "ZFAND2A",
  "gene": "UniProtKB:Q8N6M9",
  "term_label": "cytoplasm",
  "gene_name": "AN1-type zinc finger protein 2A"
}